{
  "gene": "UniProtKB:Q86VE3",
  "gene_symbol": "SATL1",
  "gene_name": "Spermidine_spermine N(1)-acetyltransferase-like protein 1",
  "term_id": "GO:0032918",
  "term_label": "spermidine acetylation"
}